{
  "term_id": "GO:0044598",
  "gene_symbol": "AKR1C2",
  "gene": "UniProtKB:P52895",
  "term_label": "doxorubicin metabolic process",
  "gene_name": "Aldo-keto reductase family 1 member C2"
}